{
  "gene_symbol": "GTF2B",
  "gene_name": "Transcription initiation factor IIB",
  "term_id": "GO:0017025",
  "term_label": "TBP-class protein binding",
  "gene": "UniProtKB:Q00403"
}